nitrite reductase (NADH) activity [GO:0106316] (molecular function) Sources: RHEA:24628 Definition: Catalysis of the reaction: NH4+ + 3 NAD+ + 2 H2O = nitrite + 3 NADH + 5 H+. Relationships: is a type of GO:0008942